{
  "gene_symbol": "EPB41L1",
  "term_id": "GO:0031032",
  "gene_name": "Band 4.1-like protein 1",
  "term_label": "actomyosin structure organization",
  "gene": "UniProtKB:Q9H4G0"
}